{
  "term_label": "endoplasmic reticulum",
  "gene": "UniProtKB:Q9H8X9",
  "gene_symbol": "ZDHHC11",
  "gene_name": "Palmitoyltransferase ZDHHC11",
  "term_id": "GO:0005783"
}